{
  "term_id": "GO:0005634",
  "gene_name": "Kelch-like protein 22",
  "gene": "UniProtKB:Q53GT1",
  "gene_symbol": "KLHL22",
  "term_label": "nucleus"
}